{
  "term_id": "GO:0002767",
  "term_label": "immune response-inhibiting cell surface receptor signaling pathway",
  "gene_name": "Killer cell immunoglobulin-like receptor 2DS3",
  "gene": "UniProtKB:Q14952",
  "gene_symbol": "KIR2DS3"
}